{
  "term_label": "iron ion binding",
  "term_id": "GO:0005506",
  "gene": "UniProtKB:Q96FX2",
  "gene_name": "Diphthamide biosynthesis protein 3",
  "gene_symbol": "DPH3"
}